extracellular matrix-cell signaling [GO:0035426] (biological process) Relationships: is a type of GO:0007154; is a type of signaling [GO:0023052] Sources: GOC:bf Definition: Any process that mediates the transfer of information between the extracellular matrix and a cell. Also known as: cell-extracellular matrix signalling, extracellular matrix-cell signalling Subtypes: extracellular matrix-granule cell signaling involved in regulation of granule cell precursor proliferation [GO:0021939], regulation of branching involved in salivary gland morphogenesis by extracellular matrix-epithelial cell signaling [GO:0060668]